{
  "gene": "UniProtKB:Q96QE4",
  "gene_symbol": "LRRC37B",
  "term_id": "UNKNOWN:0002",
  "gene_name": "Leucine-rich repeat-containing protein 37B",
  "term_label": "Unknown biological process"
}